telomeric 3' overhang formation [GO:0031860] (BP) References: PMID:16096639 Also known as: telomere 3'-end processing, telomere end processing Definition: The formation of the single stranded telomeric 3' overhang, a conserved feature that ranges in length from 12 nt in budding yeast to approximately 500 nt in humans. Relationships: is a type of DNA strand elongation [GO:0022616]; is part of telomere capping [GO:0016233]